{
  "gene_name": "Immunoglobulin lambda variable 3-25",
  "term_label": "Unknown molecular function",
  "term_id": "UNKNOWN:0001",
  "gene_symbol": "IGLV3-25",
  "gene": "UniProtKB:P01717"
}